negative regulation of inhibitory G protein-coupled receptor phosphorylation [GO:1904324] (biological process) Relationships: is a type of GO:0001933; is_a GO:0045745; is a type of GO:1904323; negatively regulates inhibitory G protein-coupled receptor phosphorylation [GO:0002030] Also known as: down regulation of inhibitory G-protein coupled receptor phosphorylation, down-regulation of inhibitory G-protein coupled receptor phosphorylation, downregulation of inhibitory G-protein coupled receptor phosphorylation, negative regulation of inhibitory G-protein coupled receptor phosphorylation, inhibition of inhibitory G-protein coupled receptor phosphorylation References: PMID:15937517 Sources: GOC:TermGenie, GO_REF:0000058 Definition: Any process that stops, prevents or reduces the frequency, rate or extent of inhibitory G protein-coupled receptor phosphorylation.